{
  "term_id": "GO:0043024",
  "gene_name": "Eukaryotic translation initiation factor 1b",
  "gene_symbol": "EIF1B",
  "term_label": "ribosomal small subunit binding",
  "gene": "UniProtKB:O60739"
}